diterpenoid biosynthetic process [GO:0016102] (biological process) Definition: The chemical reactions and pathways resulting in the formation of diterpenoid compounds, terpenoids with four isoprene units. Sources: GOC:mah, ISBN:0198547684 Subtypes: retinoic acid biosynthetic process [GO:0002138], gibberellin biosynthetic process [GO:0009686], phytol biosynthetic process [GO:0033520], vitamin A biosynthetic process [GO:0035238], tuberculosinol biosynthetic process [GO:0035440], paclitaxel biosynthetic process [GO:0042617], diterpene phytoalexin biosynthetic process [GO:0051502], GO:0140873, GO:0140879, 5alpha,9alpha,10beta-labda-8(20),13-dien-15-yl diphosphate biosynthetic process [GO:1901949], copal-8-ol diphosphate(3-) biosynthetic process [GO:1902243], cis-abienol biosynthetic process [GO:1902246] Relationships: is a type of diterpenoid metabolic process [GO:0016101]; is a type of terpenoid biosynthetic process [GO:0016114] Also known as: diterpenoid anabolism, diterpenoid biosynthesis, diterpenoid formation, diterpenoid synthesis, diterpene biosynthesis, diterpene biosynthetic process